{
  "gene_symbol": "UBP1",
  "gene_name": "Upstream-binding protein 1",
  "term_id": "GO:0005634",
  "gene": "UniProtKB:Q9NZI7",
  "term_label": "nucleus"
}